{
  "term_label": "Unknown molecular function",
  "gene_symbol": "NBEAL2",
  "gene": "UniProtKB:Q6ZNJ1",
  "gene_name": "Neurobeachin-like protein 2",
  "term_id": "UNKNOWN:0001"
}